{
  "term_id": "UNKNOWN:0002",
  "term_label": "Unknown biological process",
  "gene": "UniProtKB:Q9NQ94",
  "gene_symbol": "A1CF",
  "gene_name": "APOBEC1 complementation factor"
}